Edg-4 lysophosphatidic acid receptor binding [GO:0031757] (molecular function) Relationships: is a type of endothelial differentiation G protein-coupled receptor binding [GO:0031753] Definition: Binding to an Edg-4 lysophosphatidic acid receptor. Sources: GOC:mah, GOC:nln Also known as: LPA2 receptor binding, Edg-4 lysophosphatidic acid receptor ligand